protein phosphatase 2B binding [GO:0030346] (molecular function) Sources: GOC:jl Also known as: calcineurin binding, protein phosphatase 3 binding Definition: Binding to a protein phosphatase 2B. Relationships: is a type of protein phosphatase binding [GO:0019903]